positive regulation of phagocytosis, engulfment [GO:0060100] (biological process) Subtypes: GO:1901076 Relationships: is a type of positive regulation of phagocytosis [GO:0050766]; is a type of GO:0060099; is a type of positive regulation of membrane invagination [GO:1905155]; positively regulates phagocytosis, engulfment [GO:0006911] Sources: GOC:dph Definition: Any process that activates or increases the frequency, rate or extent of the internalization of bacteria, immune complexes and other particulate matter or of an apoptotic cell by phagocytosis.